{
  "gene_symbol": "ZNF695",
  "term_id": "GO:0000981",
  "gene_name": "Zinc finger protein 695",
  "term_label": "DNA-binding transcription factor activity, RNA polymerase II-specific",
  "gene": "UniProtKB:Q8IW36"
}